{
  "gene_name": "Hyaluronan-binding protein 2",
  "gene_symbol": "HABP2",
  "gene": "UniProtKB:Q14520",
  "term_id": "GO:0005615",
  "term_label": "extracellular space"
}